{
  "gene_symbol": "IRX2-DT",
  "gene_name": "Putative uncharacterized protein IRX2-DT",
  "term_id": "UNKNOWN:0002",
  "term_label": "Unknown biological process",
  "gene": "UniProtKB:Q86SI9"
}